{
  "term_id": "UNKNOWN:0001",
  "gene_symbol": "ZNF214",
  "gene": "UniProtKB:Q9UL59",
  "gene_name": "Zinc finger protein 214",
  "term_label": "Unknown molecular function"
}